eye blink reflex [GO:0060082] (BP) Definition: The reflex process in which a mechanical stimulus applied to the eye elicits a response of the eyelid closing. References: PMID:2913208 Sources: GOC:dph Also known as: nictitating membrane reflex Relationships: is a type of reflex [GO:0060004]